cellular detoxification [GO:1990748] (biological process) Sources: GOC:vw Subtypes: cellular detoxification of nitrogen compound [GO:0070458], cellular oxidant detoxification [GO:0098869], toxic metabolite repair [GO:0110052], cellular detoxification of aldehyde [GO:0110095], GO:0140114, cellular detoxification of metal ion [GO:0140961], cellular detoxification of sulfide [GO:0140974], cellular detoxification of acetone [GO:0140977] Relationships: is a type of GO:0009987; is_a detoxification [GO:0098754]; is part of GO:0097237 Definition: Any process carried out at the cellular level that reduces or removes the toxicity of a toxic substance. These may include transport of the toxic substance away from sensitive areas and to compartments or complexes whose purpose is sequestration of the toxic substance.